{
  "term_id": "GO:0004896",
  "gene_symbol": "IL13RA1",
  "term_label": "cytokine receptor activity",
  "gene": "UniProtKB:P78552",
  "gene_name": "Interleukin-13 receptor subunit alpha-1"
}